{
  "gene": "UniProtKB:Q9H7D0",
  "term_label": "cytoplasm",
  "gene_symbol": "DOCK5",
  "term_id": "GO:0005737",
  "gene_name": "Dedicator of cytokinesis protein 5"
}